{
  "gene": "UniProtKB:Q6PRD1",
  "gene_symbol": "GPR179",
  "term_label": "Unknown biological process",
  "term_id": "UNKNOWN:0002",
  "gene_name": "Probable G-protein coupled receptor 179"
}